{
  "gene_symbol": "CHM",
  "gene_name": "Rab proteins geranylgeranyltransferase component A 1",
  "gene": "UniProtKB:P24386",
  "term_label": "cytosol",
  "term_id": "GO:0005829"
}